plasma lipoprotein particle remodeling [GO:0034369] (biological process) Sources: GOC:BHF, GOC:expert_pt, GOC:mah, GOC:rl Definition: The acquisition, loss or modification of a protein or lipid within a plasma lipoprotein particle, including the hydrolysis of triglyceride by hepatic lipase, with the subsequent loss of free fatty acid, and the esterification of cholesterol by phosphatidylcholine-sterol O-acyltransferase (lecithin cholesterol acyltransferase; LCAT). Also known as: plasma lipoprotein particle remodelling Relationships: is a type of protein-lipid complex remodeling [GO:0034368]; is a type of plasma lipoprotein particle organization [GO:0071827]; is part of regulation of plasma lipoprotein particle levels [GO:0097006] Subtypes: GO:0034370, low-density lipoprotein particle remodeling [GO:0034374], high-density lipoprotein particle remodeling [GO:0034375], plasma lipoprotein particle oxidation [GO:0034441]